{
  "term_label": "postsynaptic density",
  "gene_symbol": "LRRC7",
  "term_id": "GO:0014069",
  "gene": "UniProtKB:Q96NW7",
  "gene_name": "Leucine-rich repeat-containing protein 7"
}